{
  "term_label": "Unknown molecular function",
  "gene": "UniProtKB:Q6RFH5",
  "gene_name": "WD repeat-containing protein 74",
  "gene_symbol": "WDR74",
  "term_id": "UNKNOWN:0001"
}